{
  "gene_name": "Inositol 1,4,5-trisphosphate receptor type 3",
  "gene_symbol": "ITPR3",
  "term_id": "GO:0030667",
  "gene": "UniProtKB:Q14573",
  "term_label": "secretory granule membrane"
}